{
  "gene_symbol": "ATG9A",
  "term_id": "GO:0034727",
  "term_label": "piecemeal microautophagy of the nucleus",
  "gene_name": "Autophagy-related protein 9A",
  "gene": "UniProtKB:Q7Z3C6"
}